seedling development [GO:0090351] (biological process) Relationships: is a type of post-embryonic development [GO:0009791] Sources: GOC:tb, PO:0007131 Definition: The process whose specific outcome is the progression of the seedling over time, beginning with seed germination and ending when the first adult leaves emerge. Regulation: regulated by regulation of seedling development [GO:1900140]